{
  "gene": "UniProtKB:Q8N9S9",
  "gene_symbol": "SNX31",
  "gene_name": "Sorting nexin-31",
  "term_id": "GO:0006886",
  "term_label": "intracellular protein transport"
}